{
  "gene_symbol": "ATP2C2",
  "gene": "UniProtKB:O75185",
  "term_label": "calcium ion transmembrane transport",
  "gene_name": "Calcium-transporting ATPase type 2C member 2",
  "term_id": "GO:0070588"
}